{
  "gene_name": "Spermatogenesis-associated protein 13",
  "term_label": "guanyl-nucleotide exchange factor activity",
  "term_id": "GO:0005085",
  "gene_symbol": "SPATA13",
  "gene": "UniProtKB:Q96N96"
}